{
  "term_label": "Unknown molecular function",
  "gene_symbol": "ZNF804A",
  "gene_name": "Zinc finger protein 804A",
  "term_id": "UNKNOWN:0001",
  "gene": "UniProtKB:Q7Z570"
}